{
  "gene_name": "Probable glutathione peroxidase 8",
  "term_id": "GO:0004601",
  "gene": "UniProtKB:Q8TED1",
  "term_label": "peroxidase activity",
  "gene_symbol": "GPX8"
}